{
  "term_label": "M band",
  "gene": "UniProtKB:Q14896",
  "term_id": "GO:0031430",
  "gene_name": "Myosin-binding protein C, cardiac-type",
  "gene_symbol": "MYBPC3"
}